{
  "gene_name": "Unconventional prefoldin RPB5 interactor 1",
  "term_id": "GO:0003682",
  "term_label": "chromatin binding",
  "gene": "UniProtKB:O94763",
  "gene_symbol": "URI1"
}